{
  "gene_symbol": "AKR1C8",
  "term_label": "Unknown cellular component",
  "term_id": "UNKNOWN:0003",
  "gene_name": "Putative aldo-keto reductase family 1 member C8",
  "gene": "UniProtKB:Q5T2L2"
}